{
  "term_id": "GO:0097116",
  "gene_name": "Neurexin-2",
  "gene": "UniProtKB:Q9P2S2",
  "term_label": "gephyrin clustering involved in postsynaptic density assembly",
  "gene_symbol": "NRXN2"
}